epithelial cell proliferation involved in salivary gland morphogenesis [GO:0060664] (biological process) Definition: The multiplication or reproduction of epithelial cells of the submandibular salivary gland, resulting in the expansion of a cell population and the shaping of the gland. References: PMID:17336109 Sources: GOC:dph Relationships: is a type of epithelial cell proliferation [GO:0050673]; is part of salivary gland morphogenesis [GO:0007435]